regulation of mRNA splicing, via spliceosome [GO:0048024] (biological process) Definition: Any process that modulates the frequency, rate or extent of mRNA splicing via a spliceosomal mechanism. Sources: GOC:jid Also known as: regulation of pre-mRNA splicing, regulation of nuclear mRNA splicing, via spliceosome, regulation of nuclear mRNA splicing via U2-type spliceosome Relationships: is a type of regulation of RNA splicing [GO:0043484]; is a type of regulation of mRNA processing [GO:0050684]; regulates mRNA splicing, via spliceosome [GO:0000398] Subtypes: regulation of alternative mRNA splicing, via spliceosome [GO:0000381], negative regulation of mRNA splicing, via spliceosome [GO:0048025], positive regulation of mRNA splicing, via spliceosome [GO:0048026], regulation of mRNA cis splicing, via spliceosome [GO:1905744]